sucrose:monoatomic cation symporter activity [GO:0009669] (molecular function) Relationships: is a type of carbohydrate:monoatomic cation symporter activity [GO:0005402]; is a type of sucrose transmembrane transporter activity [GO:0008515] Definition: Enables the transfer of a solute or solutes from one side of a membrane to the other according to the reaction: sucrose(out) + monovalent cation(out) = sucrose(in) + monovalent cation(in). Also known as: sucrose:cation symporter activity, sucrose:monovalent cation symporter activity, sucrose permease activity Sources: GOC:jy, TC:2.A.2.-.-, TC:2.A.2.4.1 Subtypes: GO:0008506